{
  "gene": "UniProtKB:O43278",
  "term_label": "serine-type endopeptidase inhibitor activity",
  "gene_name": "Kunitz-type protease inhibitor 1",
  "gene_symbol": "SPINT1",
  "term_id": "GO:0004867"
}